{
  "gene_name": "Formin-binding protein 1-like",
  "term_label": "Unknown biological process",
  "gene_symbol": "FNBP1L",
  "gene": "UniProtKB:Q5T0N5",
  "term_id": "UNKNOWN:0002"
}